{
  "gene": "UniProtKB:P20853",
  "gene_name": "Cytochrome P450 2A7",
  "term_id": "GO:0009804",
  "term_label": "coumarin metabolic process",
  "gene_symbol": "CYP2A7"
}